{
  "gene_name": "Ribosome production factor 1",
  "term_id": "GO:0000470",
  "gene_symbol": "RPF1",
  "term_label": "maturation of LSU-rRNA",
  "gene": "UniProtKB:Q9H9Y2"
}